host cell perinuclear region of cytoplasm [GO:0044220] (CC) Relationships: is a type of host cell cytoplasm part [GO:0033655] Definition: The host cell cytoplasm situated near, or occurring around, the host nucleus. Sources: GOC:rph